{
  "term_id": "GO:0006783",
  "gene": "UniProtKB:P50336",
  "term_label": "heme biosynthetic process",
  "gene_name": "Protoporphyrinogen oxidase",
  "gene_symbol": "PPOX"
}